{
  "term_id": "GO:0015629",
  "gene": "UniProtKB:Q7Z7B0",
  "term_label": "actin cytoskeleton",
  "gene_name": "Filamin-A-interacting protein 1",
  "gene_symbol": "FILIP1"
}